{
  "term_id": "GO:0005737",
  "term_label": "cytoplasm",
  "gene": "UniProtKB:P46199",
  "gene_name": "Translation initiation factor IF-2, mitochondrial",
  "gene_symbol": "MTIF2"
}